negative regulation of DNA methylation-dependent heterochromatin formation [GO:0090310] (biological process) Also known as: negative regulation of methylation-dependent chromatin silencing, negative regulation of DNA methylation-dependent heterochromatin assembly Sources: GOC:BHF Relationships: is a type of negative regulation of heterochromatin formation [GO:0031452]; negatively regulates GO:0006346 Definition: Any process that decreases the rate, frequency, or extent of DNA methylation-dependent heterochromatin formation.